{
  "gene_name": "U4_U6 small nuclear ribonucleoprotein Prp31",
  "term_id": "GO:0097526",
  "gene_symbol": "PRPF31",
  "gene": "UniProtKB:Q8WWY3",
  "term_label": "spliceosomal tri-snRNP complex"
}